{
  "gene_symbol": "S100A13",
  "term_id": "GO:0005509",
  "term_label": "calcium ion binding",
  "gene_name": "Protein S100-A13",
  "gene": "UniProtKB:Q99584"
}